{
  "gene": "UniProtKB:P0DPF3",
  "gene_symbol": "NBPF9",
  "term_label": "Unknown molecular function",
  "gene_name": "Neuroblastoma breakpoint family member 9",
  "term_id": "UNKNOWN:0001"
}